{
  "gene": "UniProtKB:Q9BX67",
  "term_id": "GO:0005886",
  "term_label": "plasma membrane",
  "gene_symbol": "JAM3",
  "gene_name": "Junctional adhesion molecule C"
}